{
  "gene": "UniProtKB:O95452",
  "term_id": "GO:0007267",
  "gene_symbol": "GJB6",
  "gene_name": "Gap junction beta-6 protein",
  "term_label": "cell-cell signaling"
}